allantoin racemase activity [GO:0047653] (molecular function) Definition: Catalysis of the reaction: (S)-(+)-allantoin = (R)-(-)-allantoin. Sources: EC:5.1.99.3, RHEA:10804 Relationships: is a type of racemase and epimerase activity [GO:0016854]